{
  "gene_name": "T cell receptor beta variable 20_OR9-2 (non-functional) (Fragment)",
  "term_id": "GO:0005886",
  "gene_symbol": "TRBV20OR9-2",
  "gene": "UniProtKB:A0A075B6H5",
  "term_label": "plasma membrane"
}